{
  "term_label": "hemopoiesis",
  "term_id": "GO:0030097",
  "gene_name": "Homeobox protein Meis1",
  "gene": "UniProtKB:O00470",
  "gene_symbol": "MEIS1"
}